{
  "term_id": "GO:0030199",
  "gene": "UniProtKB:P28300",
  "term_label": "collagen fibril organization",
  "gene_name": "Protein-lysine 6-oxidase",
  "gene_symbol": "LOX"
}